symbiont-mediated suppression of host mRNA export from nucleus [GO:0039522] (biological process) References: PMID:22334672 Sources: GOC:bf, GOC:sp Definition: A process in which a symbiont inhibits or disrupts the normal movement of mRNA from the nucleus to the cytoplasm of the host cell, leading to shutoff of host protein expression. The host is defined as the larger of the organisms involved in a symbiotic interaction. Relationships: is a type of symbiont-mediated suppression of host gene expression [GO:0039657]; is a type of symbiont-mediated perturbation of host intracellular transport [GO:0052038] Also known as: negative regulation by virus of host mRNA nuclear export, inhibition by virus of host mRNA nuclear export, inhibition of host mRNA nuclear export by virus, suppression by virus of host mRNA export from nucleus, suppression of host mRNA nuclear export by virus